{
  "gene": "UniProtKB:Q96PS8",
  "gene_symbol": "AQP10",
  "gene_name": "Aquaporin-10",
  "term_label": "glycerol transmembrane transport",
  "term_id": "GO:0015793"
}